{
  "term_id": "UNKNOWN:0001",
  "gene_name": "MAU2 chromatid cohesion factor homolog",
  "gene": "UniProtKB:Q9Y6X3",
  "gene_symbol": "MAU2",
  "term_label": "Unknown molecular function"
}